hyaline inclusion [GO:0097412] (cellular component) Definition: A glass-like, pale intracellular inclusion. Sources: NIF_Subcellular:nlx_subcell_20090104 Also known as: pale body Relationships: is_a inclusion body [GO:0016234]